{
  "term_id": "GO:0048471",
  "gene_name": "Plectin",
  "gene": "UniProtKB:Q15149",
  "gene_symbol": "PLEC",
  "term_label": "perinuclear region of cytoplasm"
}